{
  "gene_symbol": "F2RL1",
  "gene_name": "Proteinase-activated receptor 2",
  "term_label": "G protein-coupled receptor activity",
  "gene": "UniProtKB:P55085",
  "term_id": "GO:0004930"
}